{
  "gene_name": "Diacylglycerol kinase iota",
  "gene": "UniProtKB:O75912",
  "gene_symbol": "DGKI",
  "term_label": "plasma membrane",
  "term_id": "GO:0005886"
}